{
  "term_label": "external side of plasma membrane",
  "gene": "UniProtKB:Q30201",
  "gene_symbol": "HFE",
  "term_id": "GO:0009897",
  "gene_name": "Hereditary hemochromatosis protein"
}